{
  "term_label": "protein serine/threonine kinase activity",
  "gene_name": "Mitogen-activated protein kinase 7",
  "gene": "UniProtKB:Q13164",
  "term_id": "GO:0004674",
  "gene_symbol": "MAPK7"
}